{
  "term_label": "plasma membrane",
  "gene_symbol": "CALHM4",
  "term_id": "GO:0005886",
  "gene_name": "Calcium homeostasis modulator protein 4",
  "gene": "UniProtKB:Q5JW98"
}